{
  "gene": "UniProtKB:Q9UBX5",
  "term_id": "UNKNOWN:0001",
  "term_label": "Unknown molecular function",
  "gene_symbol": "FBLN5",
  "gene_name": "Fibulin-5"
}